coronary vein morphogenesis [GO:0003169] (biological process) Relationships: is_a GO:0048845; is a type of coronary vasculature morphogenesis [GO:0060977] Sources: GOC:mtg_heart Definition: The process in which the anatomical structures of veins of the heart are generated and organized.